{
  "gene_name": "Coiled-coil domain-containing protein 43",
  "gene_symbol": "CCDC43",
  "term_id": "UNKNOWN:0001",
  "gene": "UniProtKB:Q96MW1",
  "term_label": "Unknown molecular function"
}